{
  "term_id": "UNKNOWN:0001",
  "gene_symbol": "TRAV20",
  "gene": "UniProtKB:A0A0B4J274",
  "term_label": "Unknown molecular function",
  "gene_name": "T cell receptor alpha variable 20"
}